{
  "gene_symbol": "PP2D1",
  "term_id": "GO:0004722",
  "term_label": "protein serine/threonine phosphatase activity",
  "gene": "UniProtKB:A8MPX8",
  "gene_name": "Protein phosphatase 2C-like domain-containing protein 1"
}